mRNA 3'-splice site recognition [GO:0000389] (biological process) Subtypes: alignment of 3' and 5' splice sites of mRNA [GO:0034403] Definition: Recognition of the intron 3'-splice site by components of the assembling U2- or U12-type spliceosome. Sources: GOC:krc, ISBN:0879695897 Relationships: is a type of mRNA splice site recognition [GO:0006376] Also known as: nuclear mRNA 3'-splice site recognition, U12-type nuclear mRNA 3'-splice site recognition, U2-type nuclear mRNA 3'-splice site recognition